cellular response to arsenite ion [GO:1903843] (biological process) References: PMID:12106899 Sources: GOC:TermGenie, GOC:mr, GO_REF:0000071 Relationships: is a type of cellular response to arsenic-containing substance [GO:0071243]; is a type of cellular response to oxygen-containing compound [GO:1901701]; is a type of GO:1903842 Definition: Any process that results in a change in state or activity of a cell (in terms of movement, secretion, enzyme production, gene expression, etc.) as a result of an arsenite ion stimulus.